PSI associated light-harvesting complex I, LHCIb subcomplex [GO:0030084] (cellular component) Definition: A pigment protein complex that forms part of the photosystem I associated light-harvesting complex I; contains two proteins (usually about 20 kDa); has a fluorescence maximum of 730 nm. References: PMID:8825475 Relationships: is a type of PSI associated light-harvesting complex I [GO:0009518]